{
  "term_id": "UNKNOWN:0001",
  "gene_symbol": "RGS3",
  "term_label": "Unknown molecular function",
  "gene": "UniProtKB:P49796",
  "gene_name": "Regulator of G-protein signaling 3"
}